{
  "gene": "UniProtKB:A0A1W2PQC6",
  "term_id": "GO:0006369",
  "term_label": "termination of RNA polymerase II transcription",
  "gene_name": "RNA polymerase II subunit A C-terminal domain phosphatase SSU72 like protein 4",
  "gene_symbol": "SSU72L4"
}